{
  "term_label": "plasma membrane",
  "term_id": "GO:0005886",
  "gene_name": "Monocarboxylate transporter 2",
  "gene_symbol": "SLC16A7",
  "gene": "UniProtKB:O60669"
}